embryonic hemopoiesis [GO:0035162] (biological process) Sources: GOC:bf Subtypes: GO:0060215 Also known as: embryonic haematopoiesis, embryonic haemopoiesis, embryonic hematopoiesis Definition: The stages of blood cell formation that take place within the embryo. Relationships: is a type of hemopoiesis [GO:0030097]; is a type of embryonic organ development [GO:0048568]